{
  "gene_symbol": "TAS2R41",
  "gene_name": "Taste receptor type 2 member 41",
  "gene": "UniProtKB:P59536",
  "term_label": "membrane",
  "term_id": "GO:0016020"
}